pyrimidine deoxyribonucleoside interconversion [GO:0019690] (biological process) Sources: GOC:mah, ISBN:0306444747, ISBN:0471394831 Definition: The chemical reactions and pathways by which a pyrimidine deoxyribonucleoside is synthesized from another deoxyribopyrimidine nucleoside. Relationships: is a type of GO:0019689; is a type of pyrimidine deoxyribonucleoside metabolic process [GO:0046125]